{
  "gene_symbol": "KLRF1",
  "term_id": "UNKNOWN:0001",
  "gene_name": "Killer cell lectin-like receptor subfamily F member 1",
  "gene": "UniProtKB:Q9NZS2",
  "term_label": "Unknown molecular function"
}